{
  "term_label": "nucleus",
  "term_id": "GO:0005634",
  "gene": "UniProtKB:O15409",
  "gene_symbol": "FOXP2",
  "gene_name": "Forkhead box protein P2"
}